positive regulation of intracellular estrogen receptor signaling pathway [GO:0033148] (biological process) Definition: Any process that activates or increases the frequency, rate or extent of the activity of an intracellular estrogen receptor signaling pathway. Sources: GOC:mah Also known as: positive regulation of estrogen receptor signaling pathway, positive regulation of estrogen receptor signalling pathway Relationships: is a type of positive regulation of intracellular steroid hormone receptor signaling pathway [GO:0033145]; is a type of regulation of intracellular estrogen receptor signaling pathway [GO:0033146]; positively regulates GO:0030520